calcium:monoatomic cation antiporter activity [GO:0015368] (molecular function) Sources: TC:2.A.19.-.- Definition: Enables the transfer of a solute or solutes from one side of a membrane to the other according to the reaction: Ca2+(in) + cation(out) = Ca2+(out) + cation(in). Subtypes: calcium:sodium antiporter activity [GO:0005432], calcium:proton antiporter activity [GO:0015369], GO:0140983, calcium:monoatomic cation antiporter activity involved in regulation of presynaptic cytosolic calcium ion concentration [GO:1905055], calcium:monoatomic cation antiporter activity involved in regulation of postsynaptic cytosolic calcium ion concentration [GO:1905060] Also known as: calcium:cation antiporter activity Relationships: is a type of GO:0015085; is a type of metal cation:monoatomic cation antiporter activity [GO:0140828]